{
  "gene_symbol": "LINC-PINT",
  "term_id": "UNKNOWN:0003",
  "gene_name": "Transcriptional regulator PINT87aa",
  "gene": "UniProtKB:A0A455ZAR2",
  "term_label": "Unknown cellular component"
}